{
  "term_id": "GO:0005250",
  "term_label": "A-type (transient outward) potassium channel activity",
  "gene_symbol": "KCND3",
  "gene": "UniProtKB:Q9UK17",
  "gene_name": "Potassium voltage-gated channel subfamily D member 3"
}